regulation of nucleocytoplasmic transport [GO:0046822] (biological process) Definition: Any process that modulates the frequency, rate or extent of the directed movement of substances between the nucleus and the cytoplasm. Sources: GOC:bf Relationships: is_a GO:0032386; regulates nucleocytoplasmic transport [GO:0006913] Subtypes: regulation of protein import into nucleus [GO:0042306], negative regulation of nucleocytoplasmic transport [GO:0046823], positive regulation of nucleocytoplasmic transport [GO:0046824], regulation of protein export from nucleus [GO:0046825], regulation of RNA import into nucleus [GO:0046828], regulation of RNA export from nucleus [GO:0046831], regulation of ribosomal subunit export from nucleus [GO:2000200]